W-molybdopterin cofactor biosynthetic process [GO:0042047] (biological process) Definition: The chemical reactions and pathways resulting in the formation of the W-molybdopterin cofactor, essential for the catalytic activity of some enzymes. The cofactor consists of a mononuclear tungsten ion (W) coordinated by one or two molybdopterin ligands. Relationships: is a type of molybdopterin cofactor biosynthetic process [GO:0032324]; has part tungsten incorporation into tungsten-molybdopterin complex [GO:0042042] Sources: ISSN:09498257 Also known as: Moco biosynthesis, Moco biosynthetic process, W-molybdopterin cofactor anabolism, W-molybdopterin cofactor biosynthesis, W-molybdopterin cofactor formation, W-molybdopterin cofactor synthesis